regulation of GTPase activity [GO:0043087] (biological process) Subtypes: negative regulation of GTPase activity [GO:0034260], positive regulation of GTPase activity [GO:0043547], GO:1905098 Relationships: is a type of GO:0051336; regulates GTPase activity [GO:0003924] Definition: Any process that modulates the rate of GTP hydrolysis by a GTPase. Sources: GOC:jl, GOC:mah Also known as: regulation of ARF GTPase activity, regulation of Cdc42 GTPase activity, regulation of Rab GTPase activity, regulation of Rac GTPase activity, regulation of Ral GTPase activity, regulation of Ran GTPase activity, regulation of Rap GTPase activity, regulation of Ras GTPase activity, regulation of Rho GTPase activity